{
  "term_label": "G protein-coupled receptor signaling pathway",
  "gene": "UniProtKB:Q13606",
  "gene_name": "Olfactory receptor 5I1",
  "gene_symbol": "OR5I1",
  "term_id": "GO:0007186"
}